{
  "gene_name": "KICSTOR complex protein ITFG2",
  "term_label": "KICSTOR complex",
  "gene_symbol": "ITFG2",
  "term_id": "GO:0140007",
  "gene": "UniProtKB:Q969R8"
}